midbrain-hindbrain boundary maturation [GO:0021732] (biological process) Relationships: is a type of anatomical structure maturation [GO:0071695]; is part of GO:0030917 Also known as: MHB maturation, isthmus maturation Definition: A developmental process, independent of morphogenetic (shape) change, that is required for the midbrain-hindbrain boundary to attain its fully functional state. The midbrain-hindbrain domain of the embryonic brain is comprised of the mesencephalic vesicle and the first rhombencephalic vesicle at early somitogenesis stages. An organizing center at the boundary patterns the midbrain and hindbrain primordia of the neural plate. References: PMID:15541513 Sources: GOC:cls, GOC:dgh, GOC:dph, GOC:jid, GO_REF:0000021